{
  "term_label": "RNA binding",
  "term_id": "GO:0003723",
  "gene_symbol": "XRN1",
  "gene": "UniProtKB:Q8IZH2",
  "gene_name": "5'-3' exoribonuclease 1"
}